{
  "gene": "UniProtKB:P35558",
  "term_label": "phosphoenolpyruvate carboxykinase (GTP) activity",
  "term_id": "GO:0004613",
  "gene_name": "Phosphoenolpyruvate carboxykinase, cytosolic [GTP]",
  "gene_symbol": "PCK1"
}